{
  "term_label": "mitochondrion",
  "gene_symbol": "ACAD11",
  "term_id": "GO:0005739",
  "gene_name": "Acyl-CoA dehydrogenase family member 11",
  "gene": "UniProtKB:Q709F0"
}